{
  "gene_name": "Protocadherin gamma-A10",
  "term_id": "GO:0005886",
  "gene": "UniProtKB:Q9Y5H3",
  "term_label": "plasma membrane",
  "gene_symbol": "PCDHGA10"
}